peptide glutaryltransferase activity [GO:0106228] (molecular function) Definition: Catalysis of the reaction: glutaryl-CoA + L-lysyl-[protein] = CoA + H+ + N6-glutaryl-L-lysyl-[protein]. Relationships: is a type of N-acyltransferase activity [GO:0016410] References: PMID:31542297 Sources: GOC:sp Subtypes: histone glutaryltransferase activity [GO:0106229]